{
  "gene_name": "Potassium channel subfamily K member 9",
  "gene": "UniProtKB:Q9NPC2",
  "gene_symbol": "KCNK9",
  "term_label": "potassium ion leak channel activity",
  "term_id": "GO:0022841"
}